L-lysine catabolic process to acetyl-CoA via saccharopine [GO:0033512] (biological process) Also known as: L-lysine breakdown to acetyl-CoA via saccharopine, L-lysine degradation to acetyl-CoA via saccharopine Sources: GOC:mah, MetaCyc:LYSINE-DEG1-PWY Relationships: is a type of GO:0019474 Definition: The chemical reactions and pathways resulting in the breakdown of L-lysine into other compounds, including acetyl-CoA, via the intermediate saccharopine.